{
  "term_id": "GO:0006511",
  "term_label": "ubiquitin-dependent protein catabolic process",
  "gene_symbol": "NEDD4L",
  "gene": "UniProtKB:Q96PU5",
  "gene_name": "E3 ubiquitin-protein ligase NEDD4-like"
}